positive regulation of cell adhesion involved in sprouting angiogenesis [GO:0106090] (biological process) Definition: Any process that activates or increases the frequency, rate or extent of cell adhesion involved in sprouting angiogenesis. References: PMID:24177325 Sources: GOC:BHF, GOC:BHF_miRNA, GOC:rph Relationships: is a type of positive regulation of cell adhesion [GO:0045785]; is a type of regulation of cell adhesion involved in sprouting angiogenesis [GO:0106088]; RO_0002213 cell adhesion involved in sprouting angiogenesis [GO:0120078]